{
  "gene_symbol": "FOXJ2",
  "term_id": "GO:0005634",
  "gene_name": "Forkhead box protein J2",
  "term_label": "nucleus",
  "gene": "UniProtKB:Q9P0K8"
}